{
  "gene_symbol": "LLGL2",
  "term_id": "GO:0030864",
  "gene_name": "LLGL scribble cell polarity complex component 2",
  "term_label": "cortical actin cytoskeleton",
  "gene": "UniProtKB:Q6P1M3"
}